{
  "term_id": "GO:0042110",
  "gene_name": "Carcinoembryonic antigen-related cell adhesion molecule 21",
  "gene": "UniProtKB:Q3KPI0",
  "gene_symbol": "CEACAM21",
  "term_label": "T cell activation"
}